{
  "gene_name": "Alpha-1B-glycoprotein",
  "term_label": "growth hormone receptor signaling pathway",
  "gene": "UniProtKB:P04217",
  "gene_symbol": "A1BG",
  "term_id": "GO:0060396"
}